{
  "gene": "UniProtKB:Q9H845",
  "gene_symbol": "ACAD9",
  "term_label": "Unknown biological process",
  "term_id": "UNKNOWN:0002",
  "gene_name": "Complex I assembly factor ACAD9, mitochondrial"
}